{
  "gene_name": "Interactor of HORMAD1 protein 1",
  "gene_symbol": "IHO1",
  "term_label": "homologous chromosome pairing at meiosis",
  "term_id": "GO:0007129",
  "gene": "UniProtKB:Q8IYA8"
}